{
  "term_id": "GO:0019221",
  "gene_name": "Interleukin-1 beta",
  "term_label": "cytokine-mediated signaling pathway",
  "gene_symbol": "IL1B",
  "gene": "UniProtKB:P01584"
}